negative regulation of cell differentiation [GO:0045596] (biological process) Definition: Any process that stops, prevents, or reduces the frequency, rate or extent of cell differentiation. Sources: GOC:go_curators Also known as: down regulation of cell differentiation, down-regulation of cell differentiation, downregulation of cell differentiation, inhibition of cell differentiation Relationships: is a type of regulation of cell differentiation [GO:0045595]; is a type of GO:0048523; is a type of negative regulation of developmental process [GO:0051093]; RO_0002212 GO:0030154 Subtypes: maintenance of imaginal histoblast diploidy [GO:0007489], negative regulation of cell fate commitment [GO:0010454], negative regulation of epithelial to mesenchymal transition [GO:0010719], negative regulation of cell development [GO:0010721], negative regulation of macrophage derived foam cell differentiation [GO:0010745], negative regulation of epithelial cell differentiation [GO:0030857], GO:0031286, negative regulation of chondrocyte differentiation [GO:0032331], GO:0045599, negative regulation of hemocyte differentiation [GO:0045611], negative regulation of myeloid cell differentiation [GO:0045638], negative regulation of myoblast differentiation [GO:0045662], negative regulation of neuron differentiation [GO:0045665], negative regulation of osteoblast differentiation [GO:0045668], negative regulation of antipodal cell differentiation [GO:0045689], GO:0045692, negative regulation of embryo sac egg cell differentiation [GO:0045695], negative regulation of synergid differentiation [GO:0045698], negative regulation of spermatid nuclear differentiation [GO:0045701], maintenance of animal organ identity [GO:0048496], negative regulation of pigment cell differentiation [GO:0050941], negative regulation of muscle cell differentiation [GO:0051148], negative regulation of cell differentiation involved in embryonic placenta development [GO:0060806], GO:0062001, maintenance of plant organ identity [GO:0090700], negative regulation of sorocarp spore cell differentiation [GO:1901262], negative regulation of hematopoietic progenitor cell differentiation [GO:1901533], GO:1903225, negative regulation of transdifferentiation [GO:1903619], GO:1903889, GO:1904671, negative regulation of myofibroblast differentiation [GO:1904761], negative regulation of cardiocyte differentiation [GO:1905208], negative regulation of mesodermal cell differentiation [GO:1905771], negative regulation of cell differentiation involved in phenotypic switching [GO:1905916], GO:2000593, negative regulation of stem cell differentiation [GO:2000737], negative regulation of skeletal muscle cell differentiation [GO:2001015], negative regulation of tendon cell differentiation [GO:2001050], GO:2001213